{
  "term_id": "GO:0003836",
  "gene": "UniProtKB:Q16842",
  "gene_symbol": "ST3GAL2",
  "gene_name": "CMP-N-acetylneuraminate-beta-galactosamide-alpha-2,3-sialyltransferase 2",
  "term_label": "beta-galactoside (CMP) alpha-2,3-sialyltransferase activity"
}